{
  "gene_name": "MYND-type zinc finger-containing chromatin reader ZMYND8",
  "term_id": "GO:0003714",
  "term_label": "transcription corepressor activity",
  "gene_symbol": "ZMYND8",
  "gene": "UniProtKB:Q9ULU4"
}